arginine metabolic process [GO:0006525] (biological process) Relationships: is a type of alpha-amino acid metabolic process [GO:1901605] Subtypes: L-arginine biosynthetic process [GO:0006526], GO:0006527, arginine catabolic process to alanine via ornithine [GO:0010122], arginine catabolic process to spermine [GO:0019548], putrescine biosynthetic process from arginine [GO:0033388] Also known as: arginine metabolism Sources: GOC:go_curators Definition: The chemical reactions and pathways involving arginine, 2-amino-5-(carbamimidamido)pentanoic acid.